{
  "term_id": "GO:0033749",
  "gene": "UniProtKB:Q6NYC1",
  "gene_name": "Bifunctional arginine demethylase and lysyl-hydroxylase JMJD6",
  "gene_symbol": "JMJD6",
  "term_label": "histone H4R3 demethylase activity"
}